{
  "term_id": "GO:0030154",
  "gene": "UniProtKB:P36894",
  "term_label": "cell differentiation",
  "gene_name": "Bone morphogenetic protein receptor type-1A",
  "gene_symbol": "BMPR1A"
}